positive regulation of retina development in camera-type eye [GO:1902868] (biological process) Relationships: is a type of GO:0051094; is_a positive regulation of multicellular organismal process [GO:0051240]; is a type of regulation of retina development in camera-type eye [GO:1902866]; positively regulates retina development in camera-type eye [GO:0060041] References: PMID:16872597 Sources: GOC:TermGenie, GOC:mr, GO_REF:0000058 Definition: Any process that activates or increases the frequency, rate or extent of retina development in camera-type eye. Subtypes: positive regulation of neural retina development [GO:0061075] Also known as: positive regulation of retina development in camera-style eye, up regulation of retina development in camera-style eye, up regulation of retina development in camera-type eye, up-regulation of retina development in camera-style eye, up-regulation of retina development in camera-type eye, upregulation of retina development in camera-style eye, upregulation of retina development in camera-type eye, activation of retina development in camera-style eye, activation of retina development in camera-type eye, activation of retinal development, positive regulation of retinal development, up regulation of retinal development, up-regulation of retinal development, upregulation of retinal development